{
  "term_id": "UNKNOWN:0001",
  "gene": "UniProtKB:Q16586",
  "gene_symbol": "SGCA",
  "gene_name": "Alpha-sarcoglycan",
  "term_label": "Unknown molecular function"
}